{
  "term_id": "GO:0005886",
  "gene_name": "fMet-Leu-Phe receptor",
  "gene": "UniProtKB:P21462",
  "gene_symbol": "FPR1",
  "term_label": "plasma membrane"
}